{
  "gene": "UniProtKB:Q9UK13",
  "term_label": "RNA polymerase II cis-regulatory region sequence-specific DNA binding",
  "gene_name": "Zinc finger protein 221",
  "term_id": "GO:0000978",
  "gene_symbol": "ZNF221"
}